{
  "gene_symbol": "LACTB",
  "gene": "UniProtKB:P83111",
  "gene_name": "Serine beta-lactamase-like protein LACTB, mitochondrial",
  "term_id": "GO:0019216",
  "term_label": "regulation of lipid metabolic process"
}